{
  "term_label": "Unknown biological process",
  "term_id": "UNKNOWN:0002",
  "gene_name": "T cell receptor alpha joining 61 (non-functional) (Fragment)",
  "gene": "UniProtKB:A0A075B708",
  "gene_symbol": "TRAJ61"
}